response to aluminum ion [GO:0010044] (biological process) Also known as: response to aluminium ion, response to aluminum Sources: GOC:sm Subtypes: cellular response to aluminum ion [GO:0071275] Relationships: is a type of response to metal ion [GO:0010038] Definition: Any process that results in a change in state or activity of a cell or an organism (in terms of movement, secretion, enzyme production, gene expression, etc.) as a result of an aluminum ion stimulus.